{
  "term_label": "Unknown biological process",
  "gene_symbol": "COX11",
  "gene_name": "Cytochrome c oxidase assembly protein COX11, mitochondrial",
  "term_id": "UNKNOWN:0002",
  "gene": "UniProtKB:Q9Y6N1"
}